positive regulation of synaptic vesicle transport [GO:1902805] (biological process) Relationships: is a type of positive regulation of cellular process [GO:0048522]; is a type of GO:0051050; is a type of regulation of synaptic vesicle transport [GO:1902803]; positively regulates synaptic vesicle transport [GO:0048489] Subtypes: GO:1903744 Also known as: up regulation of synaptic vesicle transport, up-regulation of synaptic vesicle transport, upregulation of synaptic vesicle transport, activation of synaptic vesicle transport, activation of synaptic vesicle fission, activation of synaptic vesicle fusion, positive regulation of synaptic vesicle fission, positive regulation of synaptic vesicle fusion, up regulation of synaptic vesicle fission, up regulation of synaptic vesicle fusion, up-regulation of synaptic vesicle fission, up-regulation of synaptic vesicle fusion, upregulation of synaptic vesicle fission, upregulation of synaptic vesicle fusion Definition: Any process that activates or increases the frequency, rate or extent of synaptic vesicle transport. References: PMID:23527112 Sources: GOC:TermGenie, GOC:kmv, GO_REF:0000058